{
  "gene_name": "Calcium-binding and coiled-coil domain-containing protein 2",
  "term_id": "UNKNOWN:0001",
  "gene_symbol": "CALCOCO2",
  "gene": "UniProtKB:Q13137",
  "term_label": "Unknown molecular function"
}